plasma membrane bounded cell projection morphogenesis [GO:0120039] (biological process) Definition: The process in which the anatomical structures of a plasma membrane bounded cell projection are generated and organized. Sources: GOC:krc Relationships: is a type of cell projection morphogenesis [GO:0048858] Subtypes: cytoneme morphogenesis [GO:0003399], neuron projection morphogenesis [GO:0048812], lamellipodium morphogenesis [GO:0072673]